diphosphotransferase activity [GO:0016778] (molecular function) Definition: Catalysis of the transfer of a diphosphate group from one compound (donor) to a another (acceptor). Relationships: is a type of GO:0016772 References: PMID:1651917 Sources: GOC:jl Subtypes: 2-amino-4-hydroxy-6-hydroxymethyldihydropteridine diphosphokinase activity [GO:0003848], ribose phosphate diphosphokinase activity [GO:0004749], thiamine diphosphokinase activity [GO:0004788], GTP diphosphokinase activity [GO:0008728], nucleotide diphosphokinase activity [GO:0050148], GO:0141200